monoacylglycerol lipase activity [GO:0047372] (molecular function) Sources: RHEA:15245 Definition: Catalysis of the reaction: a monoacylglycerol + H2O = a fatty acid + glycerol + H+. Relationships: is a type of lipase activity [GO:0016298]; is a type of carboxylic ester hydrolase activity [GO:0052689] Also known as: acylglycerol lipase activity, fatty acyl monoester lipase activity, glycerol-ester acylhydrolase activity, monoacylglycerol hydrolase activity, monoacylglycerolipase activity, monoglyceridase activity, monoglyceride hydrolase activity, monoglyceride lipase activity, monoglyceridyllipase activity